{
  "term_label": "dendrite",
  "gene": "UniProtKB:O43815",
  "term_id": "GO:0030425",
  "gene_name": "Striatin",
  "gene_symbol": "STRN"
}